{
  "term_id": "GO:0035556",
  "gene": "UniProtKB:Q86XP1",
  "term_label": "intracellular signal transduction",
  "gene_symbol": "DGKH",
  "gene_name": "Diacylglycerol kinase eta"
}